{
  "term_id": "UNKNOWN:0001",
  "gene": "UniProtKB:Q69YU3",
  "gene_symbol": "ANKRD34A",
  "gene_name": "Ankyrin repeat domain-containing protein 34A",
  "term_label": "Unknown molecular function"
}